{
  "term_id": "GO:0019221",
  "gene_symbol": "STAT5B",
  "term_label": "cytokine-mediated signaling pathway",
  "gene_name": "Signal transducer and activator of transcription 5B",
  "gene": "UniProtKB:P51692"
}